{
  "term_id": "GO:0061891",
  "gene_name": "Synaptotagmin-7",
  "gene": "UniProtKB:O43581",
  "term_label": "calcium ion sensor activity",
  "gene_symbol": "SYT7"
}